{
  "gene_symbol": "AKT1",
  "term_id": "GO:0035556",
  "gene_name": "RAC-alpha serine_threonine-protein kinase",
  "term_label": "intracellular signal transduction",
  "gene": "UniProtKB:P31749"
}